positive regulation of lipoprotein lipase activity [GO:0051006] (biological process) Relationships: is a type of positive regulation of triglyceride lipase activity [GO:0061365]; positively regulates lipoprotein lipase activity [GO:0004465] Sources: GOC:ai Also known as: up regulation of lipoprotein lipase activity, up-regulation of lipoprotein lipase activity, upregulation of lipoprotein lipase activity, activation of lipoprotein lipase activity, stimulation of lipoprotein lipase activity Definition: Any process that activates or increases the activity of the enzyme lipoprotein lipase.